{
  "gene_name": "Protein-glutamine gamma-glutamyltransferase 2",
  "gene": "UniProtKB:P21980",
  "term_id": "GO:0007200",
  "gene_symbol": "TGM2",
  "term_label": "phospholipase C-activating G protein-coupled receptor signaling pathway"
}